{
  "term_id": "UNKNOWN:0003",
  "term_label": "Unknown cellular component",
  "gene_symbol": "IGHV2OR16-5",
  "gene_name": "Immunoglobulin heavy variable 2_OR16-5 (non-functional) (Fragment)",
  "gene": "UniProtKB:A0A0B4J2B6"
}